regulation of retina development in camera-type eye [GO:1902866] (biological process) Subtypes: negative regulation of retina development in camera-type eye [GO:1902867], GO:1902868 Relationships: is a type of GO:0050793; regulates retina development in camera-type eye [GO:0060041] Also known as: regulation of retina development in camera-style eye, regulation of retinal development References: PMID:16872597 Sources: GOC:TermGenie, GOC:mr, GO_REF:0000058 Definition: Any process that modulates the frequency, rate or extent of retina development in camera-type eye.